{
  "gene": "UniProtKB:P20337",
  "gene_name": "Ras-related protein Rab-3B",
  "gene_symbol": "RAB3B",
  "term_label": "synaptic vesicle",
  "term_id": "GO:0008021"
}